regulation of protein tetramerization [GO:1901090] (biological process) Definition: Any process that modulates the frequency, rate or extent of protein tetramerization. Sources: GOC:TermGenie, GOC:pm Also known as: regulation of protein tetramer assembly, regulation of protein tetramer biosynthesis, regulation of protein tetramer biosynthetic process, regulation of protein tetramer formation Relationships: is a type of regulation of protein oligomerization [GO:0032459]; regulates protein tetramerization [GO:0051262] Subtypes: negative regulation of protein tetramerization [GO:1901091], GO:1901092, GO:1901093